{
  "term_label": "Unknown biological process",
  "term_id": "UNKNOWN:0002",
  "gene_name": "Ankyrin repeat and SAM domain-containing protein 3",
  "gene": "UniProtKB:Q6ZW76",
  "gene_symbol": "ANKS3"
}